{
  "term_id": "GO:0006749",
  "gene_symbol": "HPGDS",
  "term_label": "glutathione metabolic process",
  "gene": "UniProtKB:O60760",
  "gene_name": "Hematopoietic prostaglandin D synthase"
}